{
  "term_label": "bicellular tight junction",
  "gene_symbol": "IGSF5",
  "gene": "UniProtKB:Q9NSI5",
  "gene_name": "Immunoglobulin superfamily member 5",
  "term_id": "GO:0005923"
}